{
  "term_label": "intermediate filament cytoskeleton organization",
  "gene_symbol": "PLEC",
  "gene": "UniProtKB:Q15149",
  "term_id": "GO:0045104",
  "gene_name": "Plectin"
}